phosphatidylinositol biosynthetic process [GO:0006661] (biological process) Relationships: is_a glycerophospholipid biosynthetic process [GO:0046474]; is a type of phosphatidylinositol metabolic process [GO:0046488] Subtypes: GPI anchor biosynthetic process [GO:0006506], phosphatidylinositol phosphate biosynthetic process [GO:0046854] Sources: ISBN:0198506732 Definition: The chemical reactions and pathways resulting in the formation of phosphatidylinositol, any glycophospholipid in which the sn-glycerol 3-phosphate residue is esterified to the 1-hydroxyl group of 1D-myo-inositol. Regulation: regulated by regulation of phosphatidylinositol biosynthetic process [GO:0010511]; negatively regulated by negative regulation of phosphatidylinositol biosynthetic process [GO:0010512]; positively regulated by positive regulation of phosphatidylinositol biosynthetic process [GO:0010513] Also known as: PtdIns biosynthesis, PtdIns biosynthetic process, phosphatidylinositol anabolism, phosphatidylinositol biosynthesis, phosphatidylinositol formation, phosphatidylinositol synthesis, phosphoinositide biosynthesis, phosphoinositide biosynthetic process